{
  "term_id": "GO:0009098",
  "gene_name": "Branched-chain-amino-acid aminotransferase, cytosolic",
  "gene_symbol": "BCAT1",
  "term_label": "L-leucine biosynthetic process",
  "gene": "UniProtKB:P54687"
}